gibberellin A4 carboxyl methyltransferase activity [GO:0102118] (molecular function) Definition: Catalysis of the reaction: gibberellin A4 + S-adenosyl-L-methionine = gibberellin A4 methyl ester + S-adenosyl-L-homocysteine. Sources: EC:2.1.1.276, GOC:pz Relationships: is a type of methyltransferase activity [GO:0008168]